{
  "gene_name": "STE20_SPS1-related proline-alanine-rich protein kinase",
  "term_label": "cytoplasm",
  "gene_symbol": "STK39",
  "gene": "UniProtKB:Q9UEW8",
  "term_id": "GO:0005737"
}